{
  "gene_symbol": "PAPOLB",
  "term_id": "UNKNOWN:0002",
  "gene": "UniProtKB:Q9NRJ5",
  "term_label": "Unknown biological process",
  "gene_name": "Poly(A) polymerase beta"
}